{
  "gene_name": "DNA repair protein RAD51 homolog 1",
  "term_id": "GO:0003697",
  "term_label": "single-stranded DNA binding",
  "gene_symbol": "RAD51",
  "gene": "UniProtKB:Q06609"
}